{
  "gene_name": "CDK5 regulatory subunit-associated protein 2",
  "term_id": "GO:0046600",
  "gene": "UniProtKB:Q96SN8",
  "term_label": "negative regulation of centriole replication",
  "gene_symbol": "CDK5RAP2"
}